{
  "gene_name": "Transmembrane protein 200B",
  "term_id": "UNKNOWN:0001",
  "gene_symbol": "TMEM200B",
  "gene": "UniProtKB:Q69YZ2",
  "term_label": "Unknown molecular function"
}